{
  "term_label": "ubiquitin protein ligase activity",
  "gene_symbol": "HERC6",
  "gene_name": "Probable E3 ubiquitin-protein ligase HERC6",
  "gene": "UniProtKB:Q8IVU3",
  "term_id": "GO:0061630"
}